cell envelope [GO:0030313] (cellular component) Sources: GOC:ds, GOC:mlg, http://pathmicro.med.sc.edu/fox/cell_envelope.htm Definition: An envelope that surrounds a bacterial cell and includes the cytoplasmic membrane and everything external, encompassing the periplasmic space, cell wall, and outer membrane if present. Relationships: is a type of cellular anatomical structure [GO:0110165]; has part plasma membrane [GO:0005886]